{
  "term_id": "GO:0045504",
  "gene_name": "Cytoplasmic dynein 2 light intermediate chain 1",
  "term_label": "dynein heavy chain binding",
  "gene": "UniProtKB:Q8TCX1",
  "gene_symbol": "DYNC2LI1"
}